{
  "term_label": "regulation of monoatomic cation transmembrane transport",
  "gene": "UniProtKB:Q9Y3S1",
  "gene_name": "Serine_threonine-protein kinase WNK2",
  "term_id": "GO:1904062",
  "gene_symbol": "WNK2"
}